{
  "gene_name": "Chondrolectin",
  "gene": "UniProtKB:Q9H9P2",
  "term_id": "UNKNOWN:0001",
  "gene_symbol": "CHODL",
  "term_label": "Unknown molecular function"
}